{
  "term_id": "GO:0045202",
  "gene": "UniProtKB:Q9H2B2",
  "gene_symbol": "SYT4",
  "gene_name": "Synaptotagmin-4",
  "term_label": "synapse"
}